{
  "gene": "UniProtKB:Q8NGF9",
  "gene_symbol": "OR4X2",
  "gene_name": "Olfactory receptor 4X2",
  "term_id": "GO:0005886",
  "term_label": "plasma membrane"
}